{
  "gene": "UniProtKB:Q5T653",
  "gene_symbol": "MRPL2",
  "gene_name": "Large ribosomal subunit protein uL2m",
  "term_id": "GO:0003735",
  "term_label": "structural constituent of ribosome"
}